{
  "gene_symbol": "WFDC11",
  "term_id": "GO:0045087",
  "gene_name": "Protein WFDC11",
  "gene": "UniProtKB:Q8NEX6",
  "term_label": "innate immune response"
}